{
  "gene": "UniProtKB:Q6ZVT0",
  "term_id": "UNKNOWN:0001",
  "gene_name": "Inactive polyglycylase TTLL10",
  "gene_symbol": "TTLL10",
  "term_label": "Unknown molecular function"
}